structural constituent of postsynapse [GO:0099186] (molecular function) Definition: The action of a molecule that contributes to the structural integrity of a postsynapse. Sources: GOC:dos Relationships: is a type of structural constituent of synapse [GO:0098918]; is part of postsynapse organization [GO:0099173]; BFO_0000066 postsynapse [GO:0098794] Subtypes: structural constituent of postsynaptic specialization [GO:0098879], GO:0098973, structural constituent of postsynaptic intermediate filament cytoskeleton [GO:0099184]